ATP synthesis coupled electron transport [GO:0042773] (biological process) Definition: The transfer of electrons through a series of electron donors and acceptors, generating energy that is ultimately used for synthesis of ATP. Sources: ISBN:0716731363 Relationships: is_a respiratory electron transport chain [GO:0022904]; is part of oxidative phosphorylation [GO:0006119] Subtypes: plasma membrane ATP synthesis coupled electron transport [GO:0042774], mitochondrial ATP synthesis coupled electron transport [GO:0042775]